{
  "term_id": "UNKNOWN:0002",
  "gene": "UniProtKB:Q6ZMD2",
  "gene_symbol": "SPNS3",
  "term_label": "Unknown biological process",
  "gene_name": "Protein spinster homolog 3"
}